{
  "gene_symbol": "CCDC152",
  "gene": "UniProtKB:Q4G0S7",
  "term_label": "Unknown cellular component",
  "gene_name": "Coiled-coil domain-containing protein 152",
  "term_id": "UNKNOWN:0003"
}